{
  "gene_symbol": "FRMD7",
  "gene": "UniProtKB:Q6ZUT3",
  "gene_name": "FERM domain-containing protein 7",
  "term_label": "Unknown cellular component",
  "term_id": "UNKNOWN:0003"
}